type Is terminal bouton [GO:0061177] (CC) Sources: GOC:dph, GOC:mc Relationships: is a type of type I terminal bouton [GO:0061174] Definition: Terminal inflated portion of the axon of a glutamatergic neuron, containing the specialized apparatus necessary for the phasic release neurotransmitters that will induce the contraction of muscle. Type Is terminal boutons are smaller than type Ib terminal boutons. Also known as: type Is terminal button